{
  "gene_name": "Putative uncharacterized protein LOC100506887",
  "term_id": "UNKNOWN:0003",
  "gene": "UniProtKB:Q96MF0",
  "term_label": "Unknown cellular component",
  "gene_symbol": "Q96MF0"
}